all-trans retinoic acid 3,4-desaturase activity [GO:0061898] (molecular function) Definition: Catalysis of the reaction: all-trans-retinoic acid + 2 H+ + O2 + 2 reduced [adrenodoxin] = all-trans-3,4-didehydro retinoic acid + 2 H2O + 2 oxidized [adrenodoxin]. References: PMID:27059013 Relationships: is a type of oxidoreductase activity, acting on paired donors, with incorporation or reduction of molecular oxygen [GO:0016705]